4-coumaroyl 2'-hydroxylase activity [GO:0102312] (molecular function) References: PMID:22168819, PMID:22169019 Sources: GOC:pz Relationships: is a type of 2-oxoglutarate-dependent dioxygenase activity [GO:0016706] Definition: Catalysis of the reaction: 4-coumaryl-CoA + 2-oxoglutarate + O2 = 2,4-dihydroxycinnamoyl-CoA + succinate + carbon dioxide.